{
  "gene_symbol": "NCOR1",
  "gene": "UniProtKB:O75376",
  "term_label": "chromatin",
  "term_id": "GO:0000785",
  "gene_name": "Nuclear receptor corepressor 1"
}